macroautophagy [GO:0016236] (biological process) Definition: The autophagic process that proceeds via the formation of an autophagosome. References: PMID:24366339 Also known as: autophagy, selective autophagy Relationships: is a type of autophagy [GO:0006914]; has part GO:0000045 Subtypes: mitophagy [GO:0000423], GO:0000425, ribophagy [GO:0034517], GO:0035973, nucleophagy [GO:0044804], reticulophagy [GO:0061709], glycophagy [GO:0061723], lipophagy [GO:0061724], proteaphagy [GO:0061816], GO:0062093, xenophagy [GO:0098792] Regulation: positively regulated by positive regulation of macroautophagy [GO:0016239]; regulated by regulation of macroautophagy [GO:0016241]; negatively regulated by negative regulation of macroautophagy [GO:0016242]